{
  "gene": "UniProtKB:P08758",
  "gene_name": "Annexin A5",
  "gene_symbol": "ANXA5",
  "term_label": "sarcolemma",
  "term_id": "GO:0042383"
}